{
  "gene_symbol": "FBN1",
  "term_id": "GO:0005576",
  "gene": "UniProtKB:P35555",
  "gene_name": "Fibrillin-1",
  "term_label": "extracellular region"
}